{
  "term_id": "GO:0005886",
  "gene_symbol": "OR10AD1",
  "gene_name": "Olfactory receptor 10AD1",
  "term_label": "plasma membrane",
  "gene": "UniProtKB:Q8NGE0"
}